{
  "term_label": "Unknown molecular function",
  "term_id": "UNKNOWN:0001",
  "gene": "UniProtKB:Q8NH87",
  "gene_symbol": "OR9G1",
  "gene_name": "Olfactory receptor 9G1"
}